{
  "term_id": "GO:0006888",
  "gene_symbol": "TRAPPC2",
  "gene": "UniProtKB:P0DI81",
  "gene_name": "Trafficking protein particle complex subunit 2",
  "term_label": "endoplasmic reticulum to Golgi vesicle-mediated transport"
}